cellular response to ethanol [GO:0071361] (biological process) Sources: GOC:mah Relationships: is a type of response to ethanol [GO:0045471]; is a type of cellular response to alcohol [GO:0097306] Definition: Any process that results in a change in state or activity of a cell (in terms of movement, secretion, enzyme production, gene expression, etc.) as a result of an ethanol stimulus.